{
  "gene_symbol": "COL3A1",
  "term_id": "GO:0031012",
  "gene_name": "Collagen alpha-1(III) chain",
  "gene": "UniProtKB:P02461",
  "term_label": "extracellular matrix"
}